{
  "term_label": "L-methylmalonyl-CoA metabolic process",
  "term_id": "GO:0046491",
  "gene": "UniProtKB:Q96PE7",
  "gene_symbol": "MCEE",
  "gene_name": "Methylmalonyl-CoA epimerase, mitochondrial"
}